{
  "term_label": "regulation of transcription by RNA polymerase II",
  "gene_symbol": "ZNF213",
  "gene_name": "Zinc finger protein 213",
  "gene": "UniProtKB:O14771",
  "term_id": "GO:0006357"
}